{
  "term_label": "fatty acid elongase activity",
  "gene_symbol": "ELOVL4",
  "term_id": "GO:0009922",
  "gene_name": "Elongation of very long chain fatty acids protein 4",
  "gene": "UniProtKB:Q9GZR5"
}